exon-exon junction complex binding [GO:1990448] (molecular function) Definition: Binding to an exon-exon junction complex, a protein complex deposited by the spliceosome upstream of messenger RNA exon-exon junctions. The exon-exon junction complex provides a binding platform for factors involved in mRNA export and nonsense-mediated mRNA decay. References: PMID:24967911 Sources: GOC:sart Also known as: EJC binding Relationships: is a type of protein-containing complex binding [GO:0044877]